{
  "gene_symbol": "ZDHHC9",
  "term_label": "endoplasmic reticulum",
  "term_id": "GO:0005783",
  "gene": "UniProtKB:Q9Y397",
  "gene_name": "Palmitoyltransferase ZDHHC9"
}